positive regulation of Roundabout signaling pathway [GO:0035388] (biological process) Also known as: positive regulation of Roundabout signalling pathway Definition: Any process that activates or increases the frequency, rate or extent of the Roundabout signaling pathway. Relationships: is a type of positive regulation of signal transduction [GO:0009967]; is a type of regulation of Roundabout signaling pathway [GO:0035386]; positively regulates GO:0035385 Sources: GOC:BHF